{
  "term_label": "Unknown biological process",
  "gene_symbol": "FAM220BP",
  "term_id": "UNKNOWN:0002",
  "gene": "UniProtKB:B1ANY3",
  "gene_name": "Putative protein FAM220BP"
}